{
  "term_label": "DNA binding",
  "term_id": "GO:0003677",
  "gene_symbol": "H2BC17",
  "gene_name": "Histone H2B type 1-O",
  "gene": "UniProtKB:P23527"
}